{
  "term_id": "GO:0031012",
  "term_label": "extracellular matrix",
  "gene_name": "Lysyl oxidase homolog 2",
  "gene": "UniProtKB:Q9Y4K0",
  "gene_symbol": "LOXL2"
}